{
  "gene": "UniProtKB:Q9UJ41",
  "term_id": "GO:0031267",
  "term_label": "small GTPase binding",
  "gene_symbol": "RABGEF1",
  "gene_name": "Rab5 GDP_GTP exchange factor"
}